cyanate transmembrane transporter activity [GO:0015110] (molecular function) Relationships: is a type of transmembrane transporter activity [GO:0022857]; is part of cyanate transport [GO:0015704] Sources: GOC:ai Subtypes: secondary active cyanate transmembrane transporter activity [GO:0015541] Definition: Enables the transfer of cyanate, NCO-, the anion of cyanic acid, from one side of a membrane to the other.